{
  "gene_name": "Cysteine protease ATG4D",
  "term_id": "GO:0034727",
  "term_label": "piecemeal microautophagy of the nucleus",
  "gene": "UniProtKB:Q86TL0",
  "gene_symbol": "ATG4D"
}